nerve growth factor processing [GO:0032455] (biological process) Definition: The generation of a mature nerve growth factor (NGF) by proteolysis of a precursor. Relationships: is a type of peptide hormone processing [GO:0016486] Also known as: NGF processing, beta-nerve growth factor processing References: PMID:8615794 Sources: GOC:mah